negative regulation of G0 to G1 transition [GO:0070317] (biological process) Sources: GOC:mah Definition: A cell cycle process that stops, prevents, or reduces the rate or extent of the transition from the G0 quiescent state to the G1 phase. Relationships: is a type of GO:0010948; is a type of regulation of G0 to G1 transition [GO:0070316]; negatively regulates GO:0045023 Also known as: maintenance of G0 arrest, maintenance of G0 phase, maintenance of cell cycle quiescence, maintenance of cell quiescence